Lewy body corona [GO:1990038] (cellular component) Also known as: halo Relationships: is a type of GO:0110165; is part of Lewy body [GO:0097413] Definition: The periphery of a Lewy body. In Parkinson's disease, it contains spherical accumulations of filaments arranged in a loose, radiating array. Sources: NIF_Subcellular:sao5764355747